{
  "term_label": "cytokine activity",
  "gene_symbol": "IL1A",
  "gene_name": "Interleukin-1 alpha",
  "gene": "UniProtKB:P01583",
  "term_id": "GO:0005125"
}